{
  "term_label": "Unknown cellular component",
  "gene": "UniProtKB:Q9NXU5",
  "gene_name": "ADP-ribosylation factor-like protein 15",
  "term_id": "UNKNOWN:0003",
  "gene_symbol": "ARL15"
}